{
  "gene_name": "Zinc finger protein 335",
  "gene_symbol": "ZNF335",
  "term_label": "RNA polymerase II cis-regulatory region sequence-specific DNA binding",
  "term_id": "GO:0000978",
  "gene": "UniProtKB:Q9H4Z2"
}